{
  "term_label": "cytosol",
  "term_id": "GO:0005829",
  "gene_name": "Proteasome subunit beta type-8",
  "gene": "UniProtKB:P28062",
  "gene_symbol": "PSMB8"
}